positive regulation of apoptotic process involved in development [GO:1904747] (biological process) References: PMID:22801495 Sources: GOC:TermGenie, GO_REF:0000058 Also known as: positive regulation of apoptotic cell death involved in anatomical structure development, positive regulation of apoptotic cell death involved in development of an anatomical structure, positive regulation of apoptotic process involved in anatomical structure development, positive regulation of apoptotic process involved in development of an anatomical structure, positive regulation of apoptotic programmed cell death involved in anatomical structure development, positive regulation of apoptotic programmed cell death involved in development of an anatomical structure, positive regulation of programmed cell death by apoptosis involved in anatomical structure development, positive regulation of programmed cell death by apoptosis involved in development of an anatomical structure, up regulation of apoptotic cell death involved in anatomical structure development, up regulation of apoptotic cell death involved in development of an anatomical structure, up regulation of apoptotic process involved in anatomical structure development, up regulation of apoptotic process involved in development, up regulation of apoptotic process involved in development of an anatomical structure, up regulation of apoptotic programmed cell death involved in anatomical structure development, up regulation of apoptotic programmed cell death involved in development of an anatomical structure, up regulation of programmed cell death by apoptosis involved in anatomical structure development, up regulation of programmed cell death by apoptosis involved in development of an anatomical structure, up-regulation of apoptotic cell death involved in anatomical structure development, up-regulation of apoptotic cell death involved in development of an anatomical structure, up-regulation of apoptotic process involved in anatomical structure development, up-regulation of apoptotic process involved in development, up-regulation of apoptotic process involved in development of an anatomical structure, up-regulation of apoptotic programmed cell death involved in anatomical structure development, up-regulation of apoptotic programmed cell death involved in development of an anatomical structure, up-regulation of programmed cell death by apoptosis involved in anatomical structure development, up-regulation of programmed cell death by apoptosis involved in development of an anatomical structure, upregulation of apoptotic cell death involved in anatomical structure development, upregulation of apoptotic cell death involved in development of an anatomical structure, upregulation of apoptotic process involved in anatomical structure development, upregulation of apoptotic process involved in development, upregulation of apoptotic process involved in development of an anatomical structure, upregulation of apoptotic programmed cell death involved in anatomical structure development, upregulation of apoptotic programmed cell death involved in development of an anatomical structure, upregulation of programmed cell death by apoptosis involved in anatomical structure development, upregulation of programmed cell death by apoptosis involved in development of an anatomical structure, activation of activation of apoptosis involved in anatomical structure development, activation of activation of apoptosis involved in development of an anatomical structure, activation of apoptosis involved in anatomical structure development, activation of apoptosis involved in development of an anatomical structure, activation of apoptosis signaling involved in anatomical structure development, activation of apoptosis signaling involved in development of an anatomical structure, activation of apoptotic cell death involved in anatomical structure development, activation of apoptotic cell death involved in development of an anatomical structure, activation of apoptotic process involved in anatomical structure development, activation of apoptotic process involved in development, activation of apoptotic process involved in development of an anatomical structure, activation of apoptotic program involved in anatomical structure development, activation of apoptotic program involved in development of an anatomical structure, activation of apoptotic programmed cell death involved in anatomical structure development, activation of apoptotic programmed cell death involved in development of an anatomical structure, activation of programmed cell death by apoptosis involved in anatomical structure development, activation of programmed cell death by apoptosis involved in development of an anatomical structure, activation of type I programmed cell death involved in anatomical structure development, activation of type I programmed cell death involved in development of an anatomical structure, positive regulation of activation of apoptosis involved in anatomical structure development, positive regulation of activation of apoptosis involved in development of an anatomical structure, positive regulation of apoptosis involved in anatomical structure development, positive regulation of apoptosis involved in development of an anatomical structure, positive regulation of apoptosis signaling involved in anatomical structure development, positive regulation of apoptosis signaling involved in development of an anatomical structure, positive regulation of apoptotic program involved in anatomical structure development, positive regulation of apoptotic program involved in development of an anatomical structure, positive regulation of type I programmed cell death involved in anatomical structure development, positive regulation of type I programmed cell death involved in development of an anatomical structure, up regulation of activation of apoptosis involved in anatomical structure development, up regulation of activation of apoptosis involved in development of an anatomical structure, up regulation of apoptosis involved in anatomical structure development, up regulation of apoptosis involved in development of an anatomical structure, up regulation of apoptosis signaling involved in anatomical structure development, up regulation of apoptosis signaling involved in development of an anatomical structure, up regulation of apoptotic program involved in anatomical structure development, up regulation of apoptotic program involved in development of an anatomical structure, up regulation of type I programmed cell death involved in anatomical structure development, up regulation of type I programmed cell death involved in development of an anatomical structure, up-regulation of activation of apoptosis involved in anatomical structure development, up-regulation of activation of apoptosis involved in development of an anatomical structure, up-regulation of apoptosis involved in anatomical structure development, up-regulation of apoptosis involved in development of an anatomical structure, up-regulation of apoptosis signaling involved in anatomical structure development, up-regulation of apoptosis signaling involved in development of an anatomical structure, up-regulation of apoptotic program involved in anatomical structure development, up-regulation of apoptotic program involved in development of an anatomical structure, up-regulation of type I programmed cell death involved in anatomical structure development, up-regulation of type I programmed cell death involved in development of an anatomical structure, upregulation of activation of apoptosis involved in anatomical structure development, upregulation of activation of apoptosis involved in development of an anatomical structure, upregulation of apoptosis involved in anatomical structure development, upregulation of apoptosis involved in development of an anatomical structure, upregulation of apoptosis signaling involved in anatomical structure development, upregulation of apoptosis signaling involved in development of an anatomical structure, upregulation of apoptotic program involved in anatomical structure development, upregulation of apoptotic program involved in development of an anatomical structure, upregulation of type I programmed cell death involved in anatomical structure development, upregulation of type I programmed cell death involved in development of an anatomical structure, activation of apoptosis activator activity involved in anatomical structure development, activation of apoptosis activator activity involved in development of an anatomical structure, activation of commitment to apoptosis involved in anatomical structure development, activation of commitment to apoptosis involved in development of an anatomical structure, activation of induction of apoptosis by p53 involved in anatomical structure development, activation of induction of apoptosis by p53 involved in development of an anatomical structure, activation of induction of apoptosis involved in anatomical structure development, activation of induction of apoptosis involved in development of an anatomical structure, activation of signaling (initiator) caspase activity involved in anatomical structure development, activation of signaling (initiator) caspase activity involved in development of an anatomical structure, positive regulation of apoptosis activator activity involved in anatomical structure development, positive regulation of apoptosis activator activity involved in development of an anatomical structure, positive regulation of commitment to apoptosis involved in anatomical structure development, positive regulation of commitment to apoptosis involved in development of an anatomical structure, positive regulation of induction of apoptosis by p53 involved in anatomical structure development, positive regulation of induction of apoptosis by p53 involved in development of an anatomical structure, positive regulation of induction of apoptosis involved in anatomical structure development, positive regulation of induction of apoptosis involved in development of an anatomical structure, positive regulation of signaling (initiator) caspase activity involved in anatomical structure development, positive regulation of signaling (initiator) caspase activity involved in development of an anatomical structure, up regulation of apoptosis activator activity involved in anatomical structure development, up regulation of apoptosis activator activity involved in development of an anatomical structure, up regulation of commitment to apoptosis involved in anatomical structure development, up regulation of commitment to apoptosis involved in development of an anatomical structure, up regulation of induction of apoptosis by p53 involved in anatomical structure development, up regulation of induction of apoptosis by p53 involved in development of an anatomical structure, up regulation of induction of apoptosis involved in anatomical structure development, up regulation of induction of apoptosis involved in development of an anatomical structure, up regulation of signaling (initiator) caspase activity involved in anatomical structure development, up regulation of signaling (initiator) caspase activity involved in development of an anatomical structure, up-regulation of apoptosis activator activity involved in anatomical structure development, up-regulation of apoptosis activator activity involved in development of an anatomical structure, up-regulation of commitment to apoptosis involved in anatomical structure development, up-regulation of commitment to apoptosis involved in development of an anatomical structure, up-regulation of induction of apoptosis by p53 involved in anatomical structure development, up-regulation of induction of apoptosis by p53 involved in development of an anatomical structure, up-regulation of induction of apoptosis involved in anatomical structure development, up-regulation of induction of apoptosis involved in development of an anatomical structure, up-regulation of signaling (initiator) caspase activity involved in anatomical structure development, up-regulation of signaling (initiator) caspase activity involved in development of an anatomical structure, upregulation of apoptosis activator activity involved in anatomical structure development, upregulation of apoptosis activator activity involved in development of an anatomical structure, upregulation of commitment to apoptosis involved in anatomical structure development, upregulation of commitment to apoptosis involved in development of an anatomical structure, upregulation of induction of apoptosis by p53 involved in anatomical structure development, upregulation of induction of apoptosis by p53 involved in development of an anatomical structure, upregulation of induction of apoptosis involved in anatomical structure development, upregulation of induction of apoptosis involved in development of an anatomical structure, upregulation of signaling (initiator) caspase activity involved in anatomical structure development, upregulation of signaling (initiator) caspase activity involved in development of an anatomical structure Definition: Any process that activates or increases the frequency, rate or extent of apoptotic process involved in development. Note: U4PR86 in PMID:22801495 inferred from mutant phenotype Relationships: is a type of positive regulation of apoptotic process [GO:0043065]; is a type of GO:0051094; is a type of regulation of apoptotic process involved in development [GO:1904748]; positively regulates apoptotic process involved in development [GO:1902742] Subtypes: positive regulation of B cell deletion [GO:0002869], positive regulation of nurse cell apoptotic process [GO:0045850], positive regulation of mesenchymal cell apoptotic process involved in metanephros development [GO:1900213], positive regulation of apoptotic process involved in metanephric collecting duct development [GO:1900216], GO:1900219, positive regulation of apoptotic process involved in morphogenesis [GO:1902339]